AV node cell to bundle of His cell signaling [GO:0086027] (biological process) Relationships: is a type of cell-cell signaling involved in cardiac conduction [GO:0086019]; is a type of GO:0086067 Definition: Any process that mediates the transfer of information from an AV node cardiac muscle cell to a bundle of His cardiomyocyte. Also known as: AV node cell to bundle of His cell signalling, atrioventricular node to bundle of His cell signaling Sources: GOC:BHF, GOC:mtg_cardiac_conduct_nov11